{
  "gene": "UniProtKB:Q9H2Y7",
  "gene_symbol": "ZNF106",
  "term_id": "GO:0008286",
  "gene_name": "Zinc finger protein 106",
  "term_label": "insulin receptor signaling pathway"
}